{
  "gene_symbol": "ZNF469",
  "term_label": "Unknown molecular function",
  "gene": "UniProtKB:Q96JG9",
  "term_id": "UNKNOWN:0001",
  "gene_name": "Zinc finger protein 469"
}